peptidyl-glutamine methylation [GO:0018364] (biological process) Definition: The addition of a methyl group to a glutamine residue in a protein. Sources: GOC:mah Relationships: is a type of GO:0006479